{
  "gene_symbol": "DNAAF5",
  "term_id": "GO:0003341",
  "gene_name": "Dynein axonemal assembly factor 5",
  "gene": "UniProtKB:Q86Y56",
  "term_label": "cilium movement"
}